{
  "gene_symbol": "THAP4",
  "term_label": "Unknown biological process",
  "gene_name": "Peroxynitrite isomerase THAP4",
  "term_id": "UNKNOWN:0002",
  "gene": "UniProtKB:Q8WY91"
}